{
  "gene_symbol": "RSRC2",
  "gene_name": "Arginine_serine-rich coiled-coil protein 2",
  "term_id": "UNKNOWN:0003",
  "term_label": "Unknown cellular component",
  "gene": "UniProtKB:Q7L4I2"
}